{
  "term_id": "GO:0004065",
  "gene": "UniProtKB:Q6UWY0",
  "gene_symbol": "ARSK",
  "gene_name": "Arylsulfatase K",
  "term_label": "arylsulfatase activity"
}